pyrimidine- and adenosine-specific:sodium symporter activity [GO:0015389] (molecular function) Definition: Enables the transfer of a solute or solutes from one side of a membrane to the other according to the reaction: (pyrimidine nucleoside or adenosine)(out) + Na+(out) = (pyrimidine nucleoside or adenosine)(in) + Na+(in). Sources: TC:2.A.41.2.3 Relationships: is a type of purine nucleobase transmembrane transporter activity [GO:0005345]; is a type of pyrimidine nucleobase transmembrane transporter activity [GO:0005350]; is a type of nucleoside:sodium symporter activity [GO:0005415]; is a type of nucleobase:monoatomic cation symporter activity [GO:0015391] Also known as: pyrimidine- and adenine-specific:sodium symporter activity